{
  "gene_name": "Uracil phosphoribosyltransferase homolog",
  "gene_symbol": "UPRT",
  "gene": "UniProtKB:Q96BW1",
  "term_label": "ribosylnicotinamide kinase activity",
  "term_id": "GO:0050262"
}